{
  "gene_name": "Interferon alpha-6",
  "gene": "UniProtKB:P05013",
  "term_id": "GO:0002250",
  "gene_symbol": "IFNA6",
  "term_label": "adaptive immune response"
}